{
  "gene": "UniProtKB:P13500",
  "term_label": "antimicrobial humoral immune response mediated by antimicrobial peptide",
  "term_id": "GO:0061844",
  "gene_symbol": "CCL2",
  "gene_name": "C-C motif chemokine 2"
}